starch catabolic process [GO:0005983] (biological process) Sources: GOC:ai Relationships: is a type of starch metabolic process [GO:0005982]; is a type of glucan catabolic process [GO:0009251] Also known as: starch breakdown, starch catabolism, starch degradation Regulation: regulated by regulation of starch catabolic process [GO:2000881]; negatively regulated by negative regulation of starch catabolic process [GO:2000882]; positively regulated by positive regulation of starch catabolic process [GO:2000883] Definition: The chemical reactions and pathways resulting in the breakdown of starch, the most important reserve polysaccharide in plants.